{
  "term_label": "plasma membrane",
  "gene": "UniProtKB:Q8NGQ2",
  "gene_name": "Olfactory receptor 6Q1",
  "gene_symbol": "OR6Q1",
  "term_id": "GO:0005886"
}